{
  "term_label": "phospholipid translocation",
  "gene_symbol": "ANO4",
  "gene_name": "Anoctamin-4",
  "gene": "UniProtKB:Q32M45",
  "term_id": "GO:0045332"
}